{
  "term_id": "GO:0003729",
  "gene_symbol": "SF3B1",
  "gene_name": "Splicing factor 3B subunit 1",
  "gene": "UniProtKB:O75533",
  "term_label": "mRNA binding"
}